RNA-directed DNA polymerase activity [GO:0003964] (molecular function) Relationships: is a type of DNA polymerase activity [GO:0034061]; is part of GO:0006278 Also known as: RNA-directed DNA polymerase, group II intron encoded, RNA-directed DNA polymerase, transposon encoded, DNA nucleotidyltransferase (RNA-directed) activity, RNA revertase activity, RNA-dependent DNA polymerase activity, RNA-dependent deoxyribonucleate nucleotidyltransferase activity, RNA-instructed DNA polymerase activity, RT, deoxynucleoside-triphosphate:DNA deoxynucleotidyltransferase (RNA-directed) activity, reverse transcriptase activity, revertase activity Definition: Catalysis of the reaction: a 2'-deoxyribonucleoside 5'-triphosphate + DNA(n) = diphosphate + DNA(n+1); RNA-template-directed extension of the 3'-end of a DNA strand by one deoxynucleotide at a time. Sources: EC:2.7.7.49 Subtypes: telomerase activity [GO:0003720]